positive regulation of dendritic spine morphogenesis [GO:0061003] (biological process) Relationships: is a type of positive regulation of neuron projection development [GO:0010976]; is a type of positive regulation of dendrite morphogenesis [GO:0050775]; is a type of positive regulation of dendritic spine development [GO:0060999]; is a type of GO:0061001; positively regulates dendritic spine morphogenesis [GO:0060997] Sources: GOC:dph Definition: Any process that increases the rate, frequency, or extent of dendritic spine morphogenesis, the process in which the anatomical structures of a dendritic spine are generated and organized. A dendritic spine is a protrusion from a dendrite and a specialized subcellular compartment involved in synaptic transmission.